mitochondrial malonate(1-) transmembrane transport [GO:1990558] (biological process) Definition: The process in which malonate(1-) is transported across a mitochondrial membrane, into or out of the mitochondrion. Relationships: is a type of malonic acid transmembrane transport [GO:1901553] References: PMID:10428783